{
  "gene_name": "Mimecan",
  "gene_symbol": "OGN",
  "term_label": "extracellular matrix",
  "term_id": "GO:0031012",
  "gene": "UniProtKB:P20774"
}